{
  "gene_symbol": "ATOH8",
  "gene_name": "Transcription factor ATOH8",
  "gene": "UniProtKB:Q96SQ7",
  "term_id": "GO:0009653",
  "term_label": "anatomical structure morphogenesis"
}